{
  "gene_name": "Putative serine_threonine-protein kinase PRKY",
  "gene_symbol": "PRKY",
  "term_label": "adenylate cyclase-activating G protein-coupled receptor signaling pathway",
  "gene": "UniProtKB:O43930",
  "term_id": "GO:0007189"
}